{
  "gene": "UniProtKB:Q96G21",
  "term_label": "rRNA processing",
  "gene_name": "U3 small nucleolar ribonucleoprotein protein IMP4",
  "term_id": "GO:0006364",
  "gene_symbol": "IMP4"
}